{
  "term_label": "regulation of DNA-templated transcription",
  "gene_symbol": "ZNF737",
  "gene_name": "Zinc finger protein 737",
  "gene": "UniProtKB:O75373",
  "term_id": "GO:0006355"
}